{
  "gene_name": "Fanconi anemia group D2 protein",
  "gene": "UniProtKB:Q9BXW9",
  "term_label": "interstrand cross-link repair",
  "gene_symbol": "FANCD2",
  "term_id": "GO:0036297"
}